eye development [GO:0001654] (biological process) Sources: GOC:jid, GOC:jl Subtypes: camera-type eye development [GO:0043010], GO:0048749, Bolwig's organ development [GO:0055034] Definition: The process whose specific outcome is the progression of the eye over time, from its formation to the mature structure. The eye is the organ of sight. Relationships: is a type of sensory organ development [GO:0007423]; is part of visual system development [GO:0150063]